{
  "term_label": "plasma membrane",
  "term_id": "GO:0005886",
  "gene_symbol": "CNR2",
  "gene_name": "Cannabinoid receptor 2",
  "gene": "UniProtKB:P34972"
}